alpha-amino acid catabolic process [GO:1901606] (biological process) Also known as: alpha-amino acid breakdown, alpha-amino acid catabolism, alpha-amino acid degradation Relationships: is a type of amino acid catabolic process [GO:0009063]; is a type of GO:0046395; is a type of alpha-amino acid metabolic process [GO:1901605] Definition: The chemical reactions and pathways resulting in the breakdown of an alpha-amino acid. Subtypes: GO:0006524, glycine catabolic process [GO:0006546], lysine catabolic process [GO:0006554], GO:0009093, arginine catabolic process to alanine via ornithine [GO:0010122], selenocysteine catabolic process [GO:0016261], GO:0019241, D-amino acid catabolic process [GO:0019478], arginine catabolic process to spermine [GO:0019548], glutamate catabolic process to oxaloacetate [GO:0019554], GO:0042217, GO:0043418, GO:0046948, L-amino acid catabolic process [GO:0170035], GO:1901053 Sources: GOC:TermGenie